{
  "gene": "UniProtKB:P35247",
  "gene_symbol": "SFTPD",
  "term_label": "positive regulation of phagocytosis",
  "gene_name": "Pulmonary surfactant-associated protein D",
  "term_id": "GO:0050766"
}